positive regulation of intraciliary retrograde transport [GO:1905801] (biological process) Relationships: is a type of positive regulation of intracellular transport [GO:0032388]; is_a regulation of intraciliary retrograde transport [GO:1905799]; positively regulates intraciliary retrograde transport [GO:0035721] References: PMID:27930654 Sources: GOC:TermGenie, GO_REF:0000058 Definition: Any process that activates or increases the frequency, rate or extent of intraciliary retrograde transport. Also known as: positive regulation of intraflagellar retrograde transport, up regulation of intraciliary retrograde transport, up regulation of intraflagellar retrograde transport, up-regulation of intraciliary retrograde transport, up-regulation of intraflagellar retrograde transport, upregulation of intraciliary retrograde transport, upregulation of intraflagellar retrograde transport, activation of intraciliary retrograde transport, activation of intraflagellar retrograde transport